{
  "gene_symbol": "MICALL2",
  "term_label": "actin cytoskeleton organization",
  "term_id": "GO:0030036",
  "gene_name": "MICAL-like protein 2",
  "gene": "UniProtKB:Q8IY33"
}